{
  "term_label": "signaling receptor activity",
  "gene_name": "Tumor necrosis factor receptor superfamily member EDAR",
  "gene": "UniProtKB:Q9UNE0",
  "term_id": "GO:0038023",
  "gene_symbol": "EDAR"
}